carotenoid isomerase activity [GO:0046608] (molecular function) References: PMID:11884677 Relationships: is a type of cis-trans isomerase activity [GO:0016859] Definition: Catalysis of the isomerization of poly-cis-carotenoids to all-trans-carotenoids.